{
  "gene_symbol": "DEPTOR",
  "term_id": "GO:0005096",
  "term_label": "GTPase activator activity",
  "gene": "UniProtKB:Q8TB45",
  "gene_name": "DEP domain-containing mTOR-interacting protein"
}